{
  "term_id": "GO:0042744",
  "gene": "UniProtKB:P30044",
  "gene_symbol": "PRDX5",
  "term_label": "hydrogen peroxide catabolic process",
  "gene_name": "Peroxiredoxin-5, mitochondrial"
}